{
  "gene_symbol": "CCL11",
  "term_label": "chemokine-mediated signaling pathway",
  "term_id": "GO:0070098",
  "gene_name": "Eotaxin",
  "gene": "UniProtKB:P51671"
}